{
  "gene_symbol": "APOB",
  "term_id": "GO:0042953",
  "term_label": "lipoprotein transport",
  "gene": "UniProtKB:P04114",
  "gene_name": "Apolipoprotein B-100"
}